{
  "term_label": "non-motile cilium",
  "gene": "UniProtKB:Q96M11",
  "gene_symbol": "HYLS1",
  "term_id": "GO:0097730",
  "gene_name": "Centriolar and ciliogenesis-associated protein HYLS1"
}